regulation of skeletal muscle acetylcholine-gated channel clustering [GO:1904393] (biological process) Definition: Any process that modulates the frequency, rate or extent of skeletal muscle acetylcholine-gated channel clustering. Relationships: is a type of regulation of receptor clustering [GO:1903909]; RO_0002211 skeletal muscle acetylcholine-gated channel clustering [GO:0071340] Subtypes: negative regulation of skeletal muscle acetylcholine-gated channel clustering [GO:1904394], positive regulation of skeletal muscle acetylcholine-gated channel clustering [GO:1904395] References: PMID:7722643 Sources: GOC:TermGenie, GO_REF:0000058 Also known as: regulation of skeletal muscle AChR clustering, regulation of skeletal muscle nicotinic acetylcholine receptor clustering